{
  "gene_name": "Sodium-coupled neutral amino acid transporter 5",
  "term_label": "plasma membrane",
  "gene_symbol": "SLC38A5",
  "gene": "UniProtKB:Q8WUX1",
  "term_id": "GO:0005886"
}